{
  "gene": "UniProtKB:P60059",
  "gene_name": "Protein transport protein Sec61 subunit gamma",
  "term_id": "GO:0031204",
  "gene_symbol": "SEC61G",
  "term_label": "post-translational protein targeting to membrane, translocation"
}